hinge region between urothelial plaques of apical plasma membrane [GO:0120003] (cellular component) Relationships: is_a GO:0098590; is part of apical plasma membrane [GO:0016324] Definition: A narrow rim of non-thickened membrane in between urothelial plaques in apical plasma membrane. References: PMID:21468280, PMID:21887288 Sources: GOC:krc